positive regulation of cytoskeleton organization [GO:0051495] (biological process) Sources: GOC:ai Relationships: is a type of positive regulation of organelle organization [GO:0010638]; is a type of regulation of cytoskeleton organization [GO:0051493]; positively regulates cytoskeleton organization [GO:0007010] Subtypes: GO:0030836, positive regulation of actin filament polymerization [GO:0030838], GO:0030841, positive regulation of intermediate filament depolymerization [GO:0030844], positive regulation of microtubule polymerization or depolymerization [GO:0031112], GO:0032233, GO:0046601, positive regulation of centrosome cycle [GO:0046607], positive regulation of actin nucleation [GO:0051127], positive regulation of sarcomere organization [GO:0060298], positive regulation of pseudohyphal septin ring assembly [GO:0062165], positive regulation of mitotic spindle organization [GO:0110028], GO:1903473, positive regulation of myosin II filament organization [GO:1904901], positive regulation of cardiac myofibril assembly [GO:1905306], positive regulation of spindle assembly [GO:1905832], positive regulation of cytokinesis, actomyosin contractile ring assembly [GO:2000433] Also known as: positive regulation of cytoskeleton organisation, up regulation of cytoskeleton organization, up-regulation of cytoskeleton organization, upregulation of cytoskeleton organization, activation of cytoskeleton organization, stimulation of cytoskeleton organization, positive regulation of cytoskeleton organization and biogenesis Definition: Any process that activates or increases the frequency, rate or extent of the formation, arrangement of constituent parts, or disassembly of cytoskeletal structures.